menaquinone catabolic process [GO:0042361] (biological process) Relationships: is a type of menaquinone metabolic process [GO:0009233]; is a type of ketone catabolic process [GO:0042182] Also known as: menaquinone breakdown, menaquinone catabolism, menaquinone degradation, menatetrenone catabolic process, menatetrenone catabolism, multiprenylmenaquinone catabolic process, multiprenylmenaquinone catabolism, vitamin K2 catabolic process, vitamin K2 catabolism Definition: The chemical reactions and pathways resulting in the breakdown of menaquinones, any of the quinone-derived compounds synthesized by intestinal bacteria. Structurally, menaquinones consist of a methylated naphthoquinone ring structure and side chains composed of a variable number of unsaturated isoprenoid residues. Menaquinones have vitamin K activity and are known as vitamin K2. References: PMID:37938463 Sources: GOC:jl